{
  "gene_symbol": "SPINK7",
  "gene": "UniProtKB:P58062",
  "term_label": "serine-type endopeptidase inhibitor activity",
  "term_id": "GO:0004867",
  "gene_name": "Serine protease inhibitor Kazal-type 7"
}